{
  "term_id": "GO:0006457",
  "gene": "UniProtKB:P36404",
  "term_label": "protein folding",
  "gene_symbol": "ARL2",
  "gene_name": "ADP-ribosylation factor-like protein 2"
}